{
  "term_id": "GO:0008418",
  "gene_name": "Protein N-terminal asparagine amidohydrolase",
  "gene_symbol": "NTAN1",
  "term_label": "protein-N-terminal asparagine amidohydrolase activity",
  "gene": "UniProtKB:Q96AB6"
}